{
  "gene": "UniProtKB:P32780",
  "gene_symbol": "GTF2H1",
  "term_id": "GO:0006360",
  "term_label": "transcription by RNA polymerase I",
  "gene_name": "General transcription factor IIH subunit 1"
}